L-isoleucine import across plasma membrane [GO:1903806] (biological process) Relationships: is_a organic cation transport [GO:0015695]; is a type of GO:0089718; is a type of L-alpha-amino acid transmembrane transport [GO:1902475]; is a type of isoleucine transmembrane transport [GO:1903714] References: PMID:23895341 Sources: GOC:TermGenie, GO_REF:0000075 Also known as: L-isoleucine import, isoleucine import, L-isoleucine import into cell Definition: The directed movement of L-isoleucine from outside of a cell, across the plasma membrane and into the cytosol.